{
  "term_label": "potassium ion transmembrane transport",
  "gene_symbol": "KCNC1",
  "gene": "UniProtKB:P48547",
  "term_id": "GO:0071805",
  "gene_name": "Potassium voltage-gated channel subfamily C member 1"
}